{
  "gene_symbol": "TRIM17",
  "term_label": "cytoplasm",
  "gene_name": "E3 ubiquitin-protein ligase TRIM17",
  "gene": "UniProtKB:Q9Y577",
  "term_id": "GO:0005737"
}